{
  "gene_symbol": "ZDHHC16",
  "term_label": "heart development",
  "gene_name": "Palmitoyltransferase ZDHHC16",
  "gene": "UniProtKB:Q969W1",
  "term_id": "GO:0007507"
}